{
  "term_id": "UNKNOWN:0001",
  "gene_name": "F-box_WD repeat-containing protein 8",
  "gene_symbol": "FBXW8",
  "term_label": "Unknown molecular function",
  "gene": "UniProtKB:Q8N3Y1"
}